{
  "gene": "UniProtKB:Q9BY31",
  "term_label": "nucleus",
  "gene_symbol": "ZNF717",
  "gene_name": "Zinc finger protein 717",
  "term_id": "GO:0005634"
}